{
  "gene_symbol": "PRKACG",
  "term_id": "GO:0007189",
  "term_label": "adenylate cyclase-activating G protein-coupled receptor signaling pathway",
  "gene": "UniProtKB:P22612",
  "gene_name": "cAMP-dependent protein kinase catalytic subunit gamma"
}